{
  "gene": "UniProtKB:Q8NE00",
  "gene_symbol": "TMEM104",
  "term_id": "UNKNOWN:0001",
  "gene_name": "Transmembrane protein 104",
  "term_label": "Unknown molecular function"
}